EP3 subtype prostaglandin E2 receptor binding [GO:0031866] (molecular function) Definition: Binding to an EP3 subtype prostaglandin E2 receptor. Sources: GOC:mah, GOC:nln Also known as: prostanoid EP3 receptor binding, EP3 subtype prostaglandin E2 receptor ligand Relationships: is a type of GO:0031862